{
  "term_label": "cell migration",
  "gene_name": "Protein KIBRA",
  "term_id": "GO:0016477",
  "gene_symbol": "WWC1",
  "gene": "UniProtKB:Q8IX03"
}